{
  "term_id": "GO:0002250",
  "gene_symbol": "TRAV8-1",
  "gene": "UniProtKB:A0A0A6YYK1",
  "term_label": "adaptive immune response",
  "gene_name": "T cell receptor alpha variable 8-1"
}